positive regulation of methyl-branched fatty acid biosynthetic process [GO:1902324] (BP) References: PMID:15340492 Sources: GOC:TermGenie, GOC:kmv Relationships: is a type of positive regulation of fatty acid biosynthetic process [GO:0045723]; is a type of regulation of methyl-branched fatty acid biosynthetic process [GO:1902322]; RO_0002213 GO:1902321 Also known as: positive regulation of methyl-branched fatty acid anabolism, positive regulation of methyl-branched fatty acid biosynthesis, positive regulation of methyl-branched fatty acid formation, positive regulation of methyl-branched fatty acid synthesis, up regulation of methyl-branched fatty acid anabolism, up regulation of methyl-branched fatty acid biosynthesis, up regulation of methyl-branched fatty acid biosynthetic process, up regulation of methyl-branched fatty acid formation, up regulation of methyl-branched fatty acid synthesis, up-regulation of methyl-branched fatty acid anabolism, up-regulation of methyl-branched fatty acid biosynthesis, up-regulation of methyl-branched fatty acid biosynthetic process, up-regulation of methyl-branched fatty acid formation, up-regulation of methyl-branched fatty acid synthesis, upregulation of methyl-branched fatty acid anabolism, upregulation of methyl-branched fatty acid biosynthesis, upregulation of methyl-branched fatty acid biosynthetic process, upregulation of methyl-branched fatty acid formation, upregulation of methyl-branched fatty acid synthesis, activation of methyl-branched fatty acid anabolism, activation of methyl-branched fatty acid biosynthesis, activation of methyl-branched fatty acid biosynthetic process, activation of methyl-branched fatty acid formation, activation of methyl-branched fatty acid synthesis Definition: Any process that activates or increases the frequency, rate or extent of methyl-branched fatty acid biosynthetic process.